{
  "gene_symbol": "FPR3",
  "term_label": "phospholipase C-activating G protein-coupled receptor signaling pathway",
  "term_id": "GO:0007200",
  "gene_name": "N-formyl peptide receptor 3",
  "gene": "UniProtKB:P25089"
}